{
  "gene": "UniProtKB:Q86Y13",
  "gene_symbol": "DZIP3",
  "term_id": "GO:0004842",
  "term_label": "ubiquitin-protein transferase activity",
  "gene_name": "E3 ubiquitin-protein ligase DZIP3"
}